{
  "gene_name": "Transcription factor MafB",
  "term_label": "DNA-binding transcription factor activity, RNA polymerase II-specific",
  "gene": "UniProtKB:Q9Y5Q3",
  "gene_symbol": "MAFB",
  "term_id": "GO:0000981"
}